{
  "gene_symbol": "ZNF599",
  "term_label": "nucleus",
  "term_id": "GO:0005634",
  "gene_name": "Zinc finger protein 599",
  "gene": "UniProtKB:Q96NL3"
}